{
  "term_id": "GO:0000786",
  "gene": "UniProtKB:Q9BTM1",
  "term_label": "nucleosome",
  "gene_name": "Histone H2A.J",
  "gene_symbol": "H2AJ"
}